{
  "gene": "UniProtKB:P62745",
  "gene_name": "Rho-related GTP-binding protein RhoB",
  "term_id": "GO:0005525",
  "term_label": "GTP binding",
  "gene_symbol": "RHOB"
}